L-glutamate import across plasma membrane [GO:0098712] (BP) Also known as: L-glutamate(1-) import across plasma membrane, L-glutamate import into cell, L-glutamate(1-) import into cell Sources: GOC:dos Definition: The directed movement of L-glutamate from outside of a cell, across the plasma membrane and into the cytosol. Regulation: regulated by regulation of L-glutamate import across plasma membrane [GO:0002036]; negatively regulated by GO:0002037; positively regulated by GO:0002038 Relationships: is_a L-glutamate transmembrane transport [GO:0015813]; is a type of amino acid import across plasma membrane [GO:0089718] Subtypes: glutamate reuptake [GO:0051935]